{
  "term_label": "Unknown biological process",
  "gene_symbol": "NUP43",
  "term_id": "UNKNOWN:0002",
  "gene": "UniProtKB:Q8NFH3",
  "gene_name": "Nucleoporin Nup43"
}